nitronate monooxygenase activity [GO:0018580] (molecular function) Also known as: nitronate:oxygen 2-oxidoreductase (nitrite-forming) activity, 2-nitropropane dioxygenase activity Relationships: is a type of GO:0016703 Note: Where non-covalently bound FMN is used as the cofactor, see instead 'nitronate monooxygenase (FMN-linked) activity ; GO:0036434'. Definition: Catalysis of the reaction: ethylnitronate + O2 = acetaldehyde + nitrite. Sources: EC:1.13.12.16, RHEA:28767